endothelin production [GO:1990775] (biological process) References: PMID:15560120 Relationships: is a type of cytokine production [GO:0001816] Regulation: RO_0002211 by regulation of endothelin production [GO:1904470]; negatively regulated by negative regulation of endothelin production [GO:1904471]; positively regulated by GO:1904472 Also known as: EDN1 production, EDN2 production, EDN3 production, endothelin secretion, endothelin-1 secretion, endothelin-2 production, endothelin-3 production Definition: The appearance of a endothelin due to biosynthesis or secretion following a cellular stimulus, resulting in an increase in its intracellular or extracellular levels. Endothelins are endothelium-derived vasoactive peptides involved in a variety of biological functions.